positive regulation of L-methionine import across plasma membrane [GO:1905626] (biological process) References: PMID:17556368 Sources: GOC:TermGenie, GO_REF:0000058 Definition: Any process that activates or increases the frequency, rate or extent of L-methionine import across plasma membrane. Relationships: is a type of positive regulation of organic acid transport [GO:0032892]; is a type of GO:0034764; is a type of positive regulation of amino acid transport [GO:0051957]; is a type of regulation of L-methionine import across plasma membrane [GO:1905624]; positively regulates L-methionine import across plasma membrane [GO:1905544]